{
  "gene_symbol": "SMIM19",
  "gene_name": "Small integral membrane protein 19",
  "term_id": "UNKNOWN:0001",
  "term_label": "Unknown molecular function",
  "gene": "UniProtKB:Q96E16"
}